positive regulation of protein autophosphorylation [GO:0031954] (biological process) Sources: GOC:mah Also known as: positive regulation of protein amino acid autophosphorylation, up regulation of protein amino acid autophosphorylation, up-regulation of protein amino acid autophosphorylation, upregulation of protein amino acid autophosphorylation, activation of protein amino acid autophosphorylation, stimulation of protein amino acid autophosphorylation Definition: Any process that activates or increases the frequency, rate or extent of the phosphorylation by a protein of one or more of its own residues. Relationships: is a type of positive regulation of protein phosphorylation [GO:0001934]; is a type of regulation of protein autophosphorylation [GO:0031952]; has part positive regulation of protein kinase activity [GO:0045860]; positively regulates protein autophosphorylation [GO:0046777] Subtypes: positive regulation of peptidyl-tyrosine autophosphorylation [GO:1900086]